{
  "term_id": "GO:0007189",
  "gene_symbol": "PRKACA",
  "gene": "UniProtKB:P17612",
  "gene_name": "cAMP-dependent protein kinase catalytic subunit alpha",
  "term_label": "adenylate cyclase-activating G protein-coupled receptor signaling pathway"
}